{
  "gene": "UniProtKB:A0A1B0GVV1",
  "gene_symbol": "SMIM35",
  "term_id": "UNKNOWN:0001",
  "term_label": "Unknown molecular function",
  "gene_name": "Small integral membrane protein 35"
}